L-cysteine metabolic process [GO:0046439] (biological process) Subtypes: L-cysteine catabolic process [GO:0019448] Relationships: is a type of GO:0006534; is a type of L-amino acid metabolic process [GO:0170033]; is a type of GO:0170039 Sources: GOC:ai, GOC:jsg, GOC:mah Definition: The chemical reactions and pathways involving L-cysteine, the L-enantiomer of 2-amino-3-mercaptopropanoic acid, i.e. (2R)-2-amino-3-mercaptopropanoic acid. Also known as: L-cysteine metabolism